{
  "gene_name": "Sarcoplasmic_endoplasmic reticulum calcium ATPase 1",
  "gene_symbol": "ATP2A1",
  "term_id": "GO:0070588",
  "gene": "UniProtKB:O14983",
  "term_label": "calcium ion transmembrane transport"
}